{
  "gene_name": "Cell division cycle-associated protein 7",
  "term_id": "UNKNOWN:0002",
  "gene": "UniProtKB:Q9BWT1",
  "gene_symbol": "CDCA7",
  "term_label": "Unknown biological process"
}